root hair cell development [GO:0080147] (biological process) References: PMID:19675148 Relationships: is_a cell development [GO:0048468]; is part of root hair cell differentiation [GO:0048765] Definition: The process whose specific outcome is the progression of a root hair cell over time, from its formation to the mature state.